{
  "gene": "UniProtKB:Q8IWL3",
  "gene_symbol": "HSCB",
  "gene_name": "Iron-sulfur cluster co-chaperone protein HscB",
  "term_label": "[2Fe-2S] cluster assembly",
  "term_id": "GO:0044571"
}